{
  "term_label": "extracellular space",
  "gene_name": "Keratocan",
  "gene_symbol": "KERA",
  "term_id": "GO:0005615",
  "gene": "UniProtKB:O60938"
}